regulation of mitotic cytokinesis [GO:1902412] (biological process) Subtypes: negative regulation of mitotic cytokinesis [GO:1902413], regulation of mitotic cytokinetic process [GO:1903436], positive regulation of mitotic cytokinesis [GO:1903490] Sources: GOC:TermGenie, GOC:mtg_cell_cycle Relationships: is a type of regulation of cytokinesis [GO:0032465]; regulates mitotic cytokinesis [GO:0000281] Definition: Any process that modulates the frequency, rate or extent of mitotic cytokinesis. Also known as: regulation of cytokinesis after mitosis